isoprene synthase activity [GO:0034009] (molecular function) Relationships: is a type of terpene synthase activity [GO:0010333] Sources: RHEA:13369 Also known as: ISPC, ISPS, dimethylallyl-diphosphate diphosphate-lyase (isoprene-forming) activity Definition: Catalysis of the reaction: dimethylallyl diphosphate = diphosphate + isoprene.